{
  "gene": "UniProtKB:P0CG37",
  "gene_symbol": "CFC1",
  "term_id": "GO:0005576",
  "gene_name": "Cryptic protein",
  "term_label": "extracellular region"
}